chalcone 4'-O-glucosyltransferase activity [GO:0102890] (molecular function) Sources: EC:2.4.1.286 Definition: Catalysis of the reaction: UDP-alpha-D-glucose + 2',4,4',6'-tetrahydroxychalcone = UDP + 2',4,4',6'-tetrahydroxychalcone 4'-O-beta-D-glucoside + H+. Also converts 2',3,4,4',6'-pentahydroxychalcone + UDP-alpha-D-glucose into 2',3,4,4',6'-pentahydroxychalcone 4'-O-beta-D-glucoside. Also known as: naringenin chalcone 4'-O-glucosyltransferase activity Relationships: is a type of hexosyltransferase activity [GO:0016758]